{
  "term_label": "G protein-coupled receptor binding",
  "gene": "UniProtKB:Q8WXF3",
  "gene_symbol": "RLN3",
  "gene_name": "Relaxin-3",
  "term_id": "GO:0001664"
}